{
  "gene": "UniProtKB:B0L3A2",
  "gene_name": "Dual endothelin-1_angiotensin II receptor",
  "gene_symbol": "FBXW7-AS1",
  "term_label": "Unknown molecular function",
  "term_id": "UNKNOWN:0001"
}